protein sequestering activity [GO:0140311] (molecular function) Definition: Binding to a protein to prevent it from interacting with other partners or to inhibit its localization to the area of the cell or complex where it is active. References: PMID:1493333 Subtypes: GO:0003788 Relationships: is a type of molecular sequestering activity [GO:0140313]; has part protein binding [GO:0005515]